establishment of melanosome localization [GO:0032401] (biological process) Subtypes: melanosome transport [GO:0032402] Sources: GOC:mah Also known as: establishment of melanosome localisation Definition: The directed movement of a melanosome to a specific location. Relationships: is a type of establishment of pigment granule localization [GO:0051905]; is part of GO:0032400